positive regulation of interleukin-12 production [GO:0032735] (biological process) Definition: Any process that activates or increases the frequency, rate, or extent of interleukin-12 production. Relationships: is a type of GO:0001819; is_a regulation of interleukin-12 production [GO:0032655]; positively regulates interleukin-12 production [GO:0032615] Also known as: positive regulation of IL-12 production, up regulation of interleukin-12 production, up-regulation of interleukin-12 production, upregulation of interleukin-12 production, activation of interleukin-12 production, positive regulation of interleukin-12 biosynthetic process, positive regulation of interleukin-12 secretion, stimulation of interleukin-12 production, positive regulation of CLMF production, positive regulation of NKSF production Sources: GOC:mah